{
  "gene": "UniProtKB:Q5HYJ3",
  "term_label": "Unknown molecular function",
  "gene_symbol": "FAM76B",
  "term_id": "UNKNOWN:0001",
  "gene_name": "Protein FAM76B"
}